phenanthrene-epoxide hydrolase activity [GO:0019118] (molecular function) Subtypes: phenanthrene-9,10-epoxide hydrolase activity [GO:0019119] Relationships: is_a epoxide hydrolase activity [GO:0004301] Definition: Catalysis of the reaction: a phenanthrene dioxide + H2O = a dihydrodiolphenanthrene. Sources: GOC:mah, UM-BBD_reactionID:r0535, UM-BBD_reactionID:r0536